{
  "gene": "UniProtKB:Q9HD43",
  "term_id": "UNKNOWN:0003",
  "gene_symbol": "PTPRH",
  "gene_name": "Receptor-type tyrosine-protein phosphatase H",
  "term_label": "Unknown cellular component"
}